{
  "gene_name": "Possible J 40 gene segment (Fragment)",
  "gene": "UniProtKB:A0N4X2",
  "gene_symbol": "TRAJ40",
  "term_id": "UNKNOWN:0003",
  "term_label": "Unknown cellular component"
}